{
  "term_label": "innate immune response",
  "term_id": "GO:0045087",
  "gene": "UniProtKB:Q9H1F0",
  "gene_name": "WAP four-disulfide core domain protein 10A",
  "gene_symbol": "WFDC10A"
}